{
  "term_label": "cytoskeleton organization",
  "gene_symbol": "STRIP1",
  "term_id": "GO:0007010",
  "gene": "UniProtKB:Q5VSL9",
  "gene_name": "Striatin-interacting protein 1"
}